visual system development [GO:0150063] (BP) Definition: The process whose specific outcome is the progression of the visual system over time, from its formation to the mature structure, including the eye, parts of the central nervous system (CNS) involved in processing of visual inputs, and connecting nerve pathways. Also known as: optic pathway development, visual pathway development References: PMID:15004427, PMID:20647017, PMID:22632727 Sources: GOC:aruk, GOC:bc, GOC:krc Relationships: is a type of GO:0048880